{
  "term_id": "GO:0043409",
  "gene": "UniProtKB:O14830",
  "term_label": "negative regulation of MAPK cascade",
  "gene_symbol": "PPEF2",
  "gene_name": "Serine_threonine-protein phosphatase with EF-hands 2"
}